{
  "gene_name": "Protein THEMIS",
  "gene_symbol": "THEMIS",
  "term_label": "Unknown molecular function",
  "gene": "UniProtKB:Q8N1K5",
  "term_id": "UNKNOWN:0001"
}